anthranilate N-malonyltransferase activity [GO:0047673] (molecular function) Definition: Catalysis of the reaction: anthranilate + malonyl-CoA = N-malonylanthranilate + CoA. Also known as: malonyl-CoA:anthranilate N-malonyltransferase activity Sources: EC:2.3.1.113, RHEA:17557 Relationships: is_a GO:0050735